{
  "gene_symbol": "CYBB",
  "term_id": "GO:0042554",
  "term_label": "superoxide anion generation",
  "gene": "UniProtKB:P04839",
  "gene_name": "Cytochrome b-245 heavy chain"
}